{
  "gene": "UniProtKB:Q9ULB4",
  "gene_symbol": "CDH9",
  "term_label": "adherens junction organization",
  "gene_name": "Cadherin-9",
  "term_id": "GO:0034332"
}